APC-IQGAP1-CLIP-170 complex [GO:0034746] (CC) References: PMID:15572129 Relationships: is a type of intracellular protein-containing complex [GO:0140535]; is a type of GO:1905360; is part of cell leading edge [GO:0031252] Note: Note that the gene/protein name 'APC' should not be confused with the abbreviation for 'anaphase promoting complex'. Definition: A protein complex that contains the tumor suppressor protein adenomatous polyposis coli (APC), the small GTPase Cdc42, and CLIP-170; may play a role in cytoskeleton organization and cell migration.